{
  "term_label": "membrane protein ectodomain proteolysis",
  "gene": "UniProtKB:P56817",
  "gene_name": "Beta-secretase 1",
  "term_id": "GO:0006509",
  "gene_symbol": "BACE1"
}